{
  "term_id": "GO:0000978",
  "gene": "UniProtKB:Q10587",
  "term_label": "RNA polymerase II cis-regulatory region sequence-specific DNA binding",
  "gene_symbol": "TEF",
  "gene_name": "Thyrotroph embryonic factor"
}